{
  "gene_symbol": "UCP3",
  "gene_name": "Putative mitochondrial transporter UCP3",
  "term_id": "GO:0005743",
  "term_label": "mitochondrial inner membrane",
  "gene": "UniProtKB:P55916"
}